release of sequestered calcium ion into cytosol by Golgi [GO:0061454] (biological process) Regulation: regulated by regulation of Golgi calcium ion export [GO:1901472] Also known as: Golgi calcium ion export Relationships: is a type of GO:0051209; is a type of GO:0061856 Definition: The directed movement of calcium ions (Ca2+) out of the Golgi apparatus into the cytosol. Sources: GOC:dph, GOC:tb